{
  "term_label": "Unknown cellular component",
  "gene_symbol": "HSPBAP1",
  "gene": "UniProtKB:Q96EW2",
  "gene_name": "HSPB1-associated protein 1",
  "term_id": "UNKNOWN:0003"
}